{
  "gene_symbol": "FOXA1",
  "gene": "UniProtKB:P55317",
  "gene_name": "Hepatocyte nuclear factor 3-alpha",
  "term_label": "cell differentiation",
  "term_id": "GO:0030154"
}